{
  "gene_name": "Leucine-rich repeat-containing protein 4",
  "term_label": "synaptic membrane adhesion",
  "gene_symbol": "LRRC4",
  "gene": "UniProtKB:Q9HBW1",
  "term_id": "GO:0099560"
}